{
  "term_label": "DNA-binding transcription factor activity, RNA polymerase II-specific",
  "gene_symbol": "FOXN1",
  "term_id": "GO:0000981",
  "gene_name": "Forkhead box protein N1",
  "gene": "UniProtKB:O15353"
}